{
  "gene_name": "Sentrin-specific protease 7",
  "term_id": "GO:0005737",
  "term_label": "cytoplasm",
  "gene": "UniProtKB:Q9BQF6",
  "gene_symbol": "SENP7"
}